{
  "gene_symbol": "TBP",
  "gene_name": "TATA-box-binding protein",
  "term_label": "Unknown cellular component",
  "term_id": "UNKNOWN:0003",
  "gene": "UniProtKB:P20226"
}